transport of viral material towards nucleus [GO:0075606] (biological process) Definition: The directed movement of a virus, or part of a virus, towards the host cell nucleus. The process begins after viral entry, and ends when the viral material is at the nuclear membrane. Sources: GOC:bf, GOC:jl, VZ:990 Also known as: cytoplasmic inwards viral transport, transport of viral material to nucleus, viral genome transport to host cell nucleus Note: This process does not include the viral material crossing the nuclear membrane. For transport of viral material into the nucleus, consider instead: 'viral penetration into host nucleus ; GO:0075732'. Relationships: is a type of intracellular transport of virus [GO:0075733] Subtypes: actin-dependent intracellular transport of virus towards nucleus [GO:0039680], GO:0075521